{
  "term_id": "UNKNOWN:0002",
  "gene_symbol": "GGCT",
  "gene_name": "Gamma-glutamylcyclotransferase",
  "gene": "UniProtKB:O75223",
  "term_label": "Unknown biological process"
}